peptide pheromone export by transmembrane transport [GO:0090539] (biological process) Relationships: is a type of peptide pheromone export [GO:0000770]; is a type of export across plasma membrane [GO:0140115] Also known as: peptide pheromone export by membrane transport Definition: The directed movement of a peptide pheromone across a membrane and out of a cell. Sources: GOC:al, GOC:tb, GOC:vw